{
  "gene": "UniProtKB:Q15149",
  "term_id": "GO:0005925",
  "gene_name": "Plectin",
  "term_label": "focal adhesion",
  "gene_symbol": "PLEC"
}